{
  "gene_name": "TNF receptor-associated factor 3",
  "term_id": "GO:0035591",
  "term_label": "signaling adaptor activity",
  "gene_symbol": "TRAF3",
  "gene": "UniProtKB:Q13114"
}